{
  "gene": "UniProtKB:Q14677",
  "term_id": "GO:0030276",
  "gene_name": "Clathrin interactor 1",
  "term_label": "clathrin binding",
  "gene_symbol": "CLINT1"
}